sulfide dehydrogenase activity [GO:0070225] (molecular function) Sources: RHEA:30223 Also known as: flavocytochrome c sulfide dehydrogenase activity, sulphide dehydrogenase activity Relationships: is a type of oxidoreductase activity, acting on a sulfur group of donors, cytochrome as acceptor [GO:0016669] Definition: Catalysis of the reaction: hydrogen sulfide + oxidized cytochrome c = S + reduced cytochrome c.